{
  "gene": "UniProtKB:Q96PG8",
  "gene_name": "Bcl-2-binding component 3, isoforms 3_4",
  "term_label": "positive regulation of release of cytochrome c from mitochondria",
  "term_id": "GO:0090200",
  "gene_symbol": "BBC3"
}